{
  "gene": "UniProtKB:P23786",
  "term_id": "GO:0004095",
  "term_label": "carnitine O-palmitoyltransferase activity",
  "gene_name": "Carnitine O-palmitoyltransferase 2, mitochondrial",
  "gene_symbol": "CPT2"
}